tRNA (guanine(18)-2'-O)-methyltransferase activity [GO:0141100] (molecular function) Definition: Catalysis of the reaction: S-adenosyl-L-methionine + guanosine 18 in tRNA= S-adenosyl-L-homocysteine + 2'-O-methylguanosine 18 in tRNA + H+. Relationships: is a type of tRNA (guanine) methyltransferase activity [GO:0016423] References: PMID:25404562 Also known as: tRNA (guanosine(18)-2'-O)-methyltransferase activity